{
  "gene": "UniProtKB:Q96IK1",
  "gene_symbol": "BOD1",
  "term_label": "Unknown biological process",
  "term_id": "UNKNOWN:0002",
  "gene_name": "Biorientation of chromosomes in cell division protein 1"
}